{
  "term_label": "calcium ion transmembrane transport",
  "gene_symbol": "P2RX7",
  "gene": "UniProtKB:Q99572",
  "term_id": "GO:0070588",
  "gene_name": "P2X purinoceptor 7"
}